{
  "gene_name": "DnaJ homolog subfamily C member 30, mitochondrial",
  "gene": "UniProtKB:Q96LL9",
  "gene_symbol": "DNAJC30",
  "term_id": "UNKNOWN:0003",
  "term_label": "Unknown cellular component"
}